{
  "term_label": "GTPase activator activity",
  "gene": "UniProtKB:Q96HU1",
  "gene_symbol": "SGSM3",
  "gene_name": "Small G protein signaling modulator 3",
  "term_id": "GO:0005096"
}